{
  "term_label": "Unknown molecular function",
  "gene_name": "Translocator protein",
  "gene": "UniProtKB:P30536",
  "term_id": "UNKNOWN:0001",
  "gene_symbol": "TSPO"
}